regulation of chemokine (C-C motif) ligand 6 production [GO:0035531] (biological process) Relationships: is a type of regulation of chemokine production [GO:0032642]; RO_0002211 chemokine (C-C motif) ligand 6 production [GO:0035530] Subtypes: negative regulation of chemokine (C-C motif) ligand 6 production [GO:0035532], positive regulation of chemokine (C-C motif) ligand 6 production [GO:0035533] Also known as: regulation of CCL6 production, chemokine (C-C motif) ligand 6 secretion, regulation of chemokine (C-C motif) ligand 6 secretion Sources: GOC:add, GOC:bf Definition: Any process that modulates the frequency, rate, or extent of production of chemokine (C-C motif) ligand 6 (CCL6).